{
  "gene": "UniProtKB:Q8NGJ4",
  "term_label": "plasma membrane",
  "gene_name": "Olfactory receptor 52E2",
  "term_id": "GO:0005886",
  "gene_symbol": "OR52E2"
}